{
  "term_label": "endoplasmic reticulum to Golgi vesicle-mediated transport",
  "gene": "UniProtKB:O43617",
  "gene_symbol": "TRAPPC3",
  "term_id": "GO:0006888",
  "gene_name": "Trafficking protein particle complex subunit 3"
}